magnetoreception by sensory perception of electrical stimulus [GO:0050978] (biological process) Relationships: is a type of sensory perception of electrical stimulus [GO:0050952]; is_a magnetoreception [GO:0050958] References: PMID:15886990 Sources: GOC:ai, Wikipedia:Magnetoception Also known as: magnetoreception by electrical stimulus, magnetoreception through electrical stimulus, magnetoreception, sensory perception of electrical stimulus, magnetoreception, using electrical stimulus Definition: The series of events required for an organism to receive an electrical stimulus relating to a magnetic field, convert it to a molecular signal, and recognize and characterize the signal. Movement in a magnetic field results in an induced electric field, which can be perceived by organisms such as elasmobranch fish.